acetoacetyl-CoA hydrolase activity [GO:0047603] (molecular function) Also known as: acetoacetyl CoA deacylase activity, acetoacetyl coenzyme A deacylase activity, acetoacetyl coenzyme A hydrolase activity Relationships: is a type of acyl-CoA hydrolase activity [GO:0016289] Sources: EC:3.1.2.11, RHEA:15673 Definition: Catalysis of the reaction: acetoacetyl-CoA + H2O = acetoacetate + CoA + H+.